positive regulation of intrinsic apoptotic signaling pathway in response to hydrogen peroxide [GO:1903752] (biological process) Relationships: is a type of positive regulation of hydrogen peroxide-mediated programmed cell death [GO:1901300]; is a type of positive regulation of oxidative stress-induced intrinsic apoptotic signaling pathway [GO:1902177]; is a type of regulation of intrinsic apoptotic signaling pathway in response to hydrogen peroxide [GO:1903750]; positively regulates intrinsic apoptotic signaling pathway in response to hydrogen peroxide [GO:0036481] Also known as: positive regulation of hydrogen peroxide-induced intrinsic apoptotic signaling pathway, positive regulation of intrinsic apoptotic signaling pathway in response to H2O2, up regulation of hydrogen peroxide-induced intrinsic apoptotic signaling pathway, up regulation of intrinsic apoptotic signaling pathway in response to H2O2, up regulation of intrinsic apoptotic signaling pathway in response to hydrogen peroxide, up-regulation of hydrogen peroxide-induced intrinsic apoptotic signaling pathway, up-regulation of intrinsic apoptotic signaling pathway in response to H2O2, up-regulation of intrinsic apoptotic signaling pathway in response to hydrogen peroxide, upregulation of hydrogen peroxide-induced intrinsic apoptotic signaling pathway, upregulation of intrinsic apoptotic signaling pathway in response to H2O2, upregulation of intrinsic apoptotic signaling pathway in response to hydrogen peroxide, activation of hydrogen peroxide-induced intrinsic apoptotic signaling pathway, activation of intrinsic apoptotic signaling pathway in response to H2O2, activation of intrinsic apoptotic signaling pathway in response to hydrogen peroxide, activation of H2O2-induced intrinsic apoptotic signaling pathway, positive regulation of H2O2-induced intrinsic apoptotic signaling pathway, up regulation of H2O2-induced intrinsic apoptotic signaling pathway, up-regulation of H2O2-induced intrinsic apoptotic signaling pathway, upregulation of H2O2-induced intrinsic apoptotic signaling pathway Definition: Any process that activates or increases the frequency, rate or extent of intrinsic apoptotic signaling pathway in response to hydrogen peroxide. References: PMID:18681888 Sources: GOC:TermGenie, GO_REF:0000058